interleukin-18 receptor activity [GO:0042008] (molecular function) Definition: Combining with interleukin-18 and transmitting the signal from one side of the membrane to the other to initiate a change in cell activity. Relationships: is a type of cytokine receptor activity [GO:0004896]; is part of interleukin-18-mediated signaling pathway [GO:0035655]; has part GO:0042007 Also known as: IL-18 receptor activity, IL-18R Sources: GOC:jl, GOC:signaling